{
  "gene_symbol": "HLA-DOA",
  "gene_name": "HLA class II histocompatibility antigen, DO alpha chain",
  "term_id": "GO:0019886",
  "term_label": "antigen processing and presentation of exogenous peptide antigen via MHC class II",
  "gene": "UniProtKB:P06340"
}